negative regulation of membrane depolarization during cardiac muscle cell action potential [GO:1900826] (biological process) Also known as: down regulation of membrane depolarization during cardiac muscle cell action potential, down-regulation of membrane depolarization during of cardiac muscle cell action potential, downregulation of membrane depolarization during cardiac muscle cell action potential, inhibition of membrane depolarization during cardiac muscle cell action potential Relationships: is a type of regulation of membrane depolarization during cardiac muscle cell action potential [GO:1900825]; is a type of negative regulation of membrane depolarization [GO:1904180]; negatively regulates GO:0086012 Sources: GOC:BHF, GOC:TermGenie, GOC:mtg_cardiac_conduct_nov11 Definition: Any process that stops, prevents or reduces the frequency, rate or extent of membrane depolarization during a cardiac muscle cell action potential. Subtypes: GO:1905028